{
  "gene_symbol": "HEY1",
  "gene_name": "Hairy_enhancer-of-split related with YRPW motif protein 1",
  "gene": "UniProtKB:Q9Y5J3",
  "term_id": "GO:0050767",
  "term_label": "regulation of neurogenesis"
}